{
  "term_id": "UNKNOWN:0001",
  "term_label": "Unknown molecular function",
  "gene": "UniProtKB:Q6NUJ2",
  "gene_symbol": "C11orf87",
  "gene_name": "Uncharacterized protein C11orf87"
}